{
  "gene": "UniProtKB:A0A075B6V5",
  "gene_symbol": "TRAV36DV7",
  "gene_name": "T cell receptor alpha variable 36_delta variable 7",
  "term_label": "Unknown cellular component",
  "term_id": "UNKNOWN:0003"
}